{
  "gene_symbol": "FAM236C",
  "gene_name": "Protein FAM236C",
  "gene": "UniProtKB:P0DP71",
  "term_id": "UNKNOWN:0002",
  "term_label": "Unknown biological process"
}